{
  "term_label": "cyclin-dependent protein serine/threonine kinase regulator activity",
  "gene": "UniProtKB:Q8WWL7",
  "gene_symbol": "CCNB3",
  "gene_name": "G2_mitotic-specific cyclin-B3",
  "term_id": "GO:0016538"
}